{
  "gene_name": "3-keto-steroid reductase_17-beta-hydroxysteroid dehydrogenase 7",
  "gene": "UniProtKB:P56937",
  "gene_symbol": "HSD17B7",
  "term_label": "5-alpha-androstane-3-beta,17-beta-diol dehydrogenase (NADP+) activity",
  "term_id": "GO:0047024"
}